{
  "gene_symbol": "CRNKL1",
  "term_id": "GO:0000398",
  "gene": "UniProtKB:Q9BZJ0",
  "term_label": "mRNA splicing, via spliceosome",
  "gene_name": "Crooked neck-like protein 1"
}